mitochondrial small ribosomal subunit assembly [GO:0180026] (biological process) Relationships: is a type of GO:0000028; is part of GO:0061668 References: PMID:30467428 Definition: The aggregation, arrangement and bonding together of a set of components to form a mitochondrial small ribosomal subunit.